{
  "gene_symbol": "LTB",
  "term_label": "cell surface receptor signaling pathway",
  "gene": "UniProtKB:Q06643",
  "gene_name": "Lymphotoxin-beta",
  "term_id": "GO:0007166"
}